{
  "gene_name": "Annexin A9",
  "term_id": "GO:0005634",
  "gene": "UniProtKB:O76027",
  "gene_symbol": "ANXA9",
  "term_label": "nucleus"
}